{
  "term_id": "GO:0006107",
  "term_label": "oxaloacetate metabolic process",
  "gene_name": "Malate dehydrogenase, cytoplasmic",
  "gene_symbol": "MDH1",
  "gene": "UniProtKB:P40925"
}